{
  "gene_symbol": "DYNC1I1",
  "term_label": "dynein heavy chain binding",
  "term_id": "GO:0045504",
  "gene": "UniProtKB:O14576",
  "gene_name": "Cytoplasmic dynein 1 intermediate chain 1"
}